{
  "gene_name": "Zinc finger protein 354A",
  "gene": "UniProtKB:O60765",
  "term_id": "GO:0006357",
  "term_label": "regulation of transcription by RNA polymerase II",
  "gene_symbol": "ZNF354A"
}